activation of protein kinase B activity [GO:0032148] (biological process) Relationships: is a type of GO:0032147 Sources: GOC:pg Definition: Any process that initiates the activity of the inactive enzyme protein kinase B. Also known as: protein kinase B activation